{
  "gene_name": "Gamma-parvin",
  "term_id": "GO:0034446",
  "gene_symbol": "PARVG",
  "gene": "UniProtKB:Q9HBI0",
  "term_label": "substrate adhesion-dependent cell spreading"
}